{
  "gene": "UniProtKB:P13500",
  "term_id": "GO:0070098",
  "gene_symbol": "CCL2",
  "gene_name": "C-C motif chemokine 2",
  "term_label": "chemokine-mediated signaling pathway"
}